{
  "gene": "UniProtKB:Q8NBL1",
  "gene_name": "Protein O-glucosyltransferase 1",
  "term_label": "UDP-glucosyltransferase activity",
  "gene_symbol": "POGLUT1",
  "term_id": "GO:0035251"
}